negative regulation of extracellular matrix assembly [GO:1901202] (biological process) Relationships: is a type of GO:1901201; is a type of negative regulation of extracellular matrix organization [GO:1903054]; negatively regulates extracellular matrix assembly [GO:0085029] Also known as: down regulation of extracellular matrix assembly, down-regulation of extracellular matrix assembly, downregulation of extracellular matrix assembly, inhibition of extracellular matrix assembly Subtypes: negative regulation of basement membrane assembly involved in embryonic body morphogenesis [GO:1904260] Sources: GOC:BHF, GOC:TermGenie Definition: Any process that stops, prevents or reduces the frequency, rate or extent of extracellular matrix assembly.